virion assembly [GO:0019068] (biological process) Definition: A late phase of the viral life cycle during which all the components necessary for the formation of a mature virion collect at a particular site in the cell and the basic structure of the virus particle is formed. Sources: ISBN:0121585336 Also known as: viral assembly, viral particle assembly, virion assembly and maintenance, virion organization, virus assembly, virus particle assembly, bacteriophage assembly, phage assembly Relationships: is a type of viral process [GO:0016032]; is part of GO:0019058